{
  "gene": "UniProtKB:Q99584",
  "term_label": "perinuclear region of cytoplasm",
  "gene_symbol": "S100A13",
  "gene_name": "Protein S100-A13",
  "term_id": "GO:0048471"
}